{
  "term_id": "GO:0042981",
  "term_label": "regulation of apoptotic process",
  "gene_symbol": "USP42",
  "gene_name": "Ubiquitin carboxyl-terminal hydrolase 42",
  "gene": "UniProtKB:Q9H9J4"
}